GAC codon-amino acid adaptor activity [GO:0033458] (molecular function) Note: Note that in the standard genetic code, GAC codes for aspartic acid. Relationships: is a type of GO:0030533 Also known as: aspartic acid tRNA Definition: A triplet codon-amino acid adaptor activity that recognizes a GAC codon. Sources: GOC:mah